protein localization to pericentriolar material [GO:1905793] (biological process) Definition: A process in which a protein is transported to, or maintained in, a location within a pericentriolar material. Also known as: protein localisation in pericentriolar material, protein localisation to pericentriolar material, protein localization in pericentriolar material References: PMID:21694707, PMID:24385583 Sources: GOC:TermGenie, GO_REF:0000087 Relationships: is a type of protein localization to centrosome [GO:0071539]